(+)-abscisic acid D-glucopyranosyl ester transmembrane transport [GO:1902418] (BP) Definition: The process in which (+)-abscisic acid D-glucopyranosyl este is transported across a membrane. Also known as: ABA-GE transmembrane transport, abscisic acid glucosyl ester transmembrane transport References: PMID:24028845 Sources: GOC:TermGenie Relationships: is a type of glucoside transport [GO:0042946]; is a type of transmembrane transport [GO:0055085]